beta,beta-carotene-9',10'-cleaving oxygenase activity [GO:0102076] (molecular function) Sources: EC:1.13.11.71, GOC:pz Relationships: is a type of oxidoreductase activity, acting on single donors with incorporation of molecular oxygen, incorporation of two atoms of oxygen [GO:0016702] Definition: Catalysis of the reaction: beta-carotene + O2 = 10'-apo-beta-carotenal + beta-ionone.